palmitoyl-(protein) hydrolase activity [GO:0008474] (molecular function) Definition: Catalysis of the reaction: palmitoyl-protein + H2O = palmitate + protein. Also known as: palmitoyl-[protein] hydrolase, palmitoyl-protein hydrolase activity, palmitoyl-protein thioesterase activity, palmitoyl-protein thiolesterase activity Relationships: is a type of GO:0016790; is a type of palmitoyl hydrolase activity [GO:0098599]; is a type of catalytic activity, acting on a protein [GO:0140096] Sources: EC:3.1.2.22